definitive hemopoiesis [GO:0060216] (BP) Also known as: definitive haemopoiesis, definitive hematopoiesis, definitive haematopoiesis Relationships: is a type of hemopoiesis [GO:0030097] Definition: A second wave of blood cell production that, in vertebrates, generates long-term hemopoietic stem cells that continuously provide erythroid, myeloid and lymphoid lineages throughout adulthood. References: PMID:15378083, PMID:15617691 Sources: GOC:bf, GOC:dph